{
  "gene_symbol": "CELF5",
  "term_label": "nucleus",
  "term_id": "GO:0005634",
  "gene_name": "CUGBP Elav-like family member 5",
  "gene": "UniProtKB:Q8N6W0"
}